establishment of centrosome localization [GO:0051660] (biological process) Definition: The directed movement of the centrosome to a specific location. Sources: GOC:ai Also known as: centrosome positioning, establishment of centrosome localisation Relationships: is a type of centrosome localization [GO:0051642]; is a type of GO:0051649; is a type of establishment of organelle localization [GO:0051656]